chloroplast photosystem II binding [GO:0062068] (molecular function) Definition: Binding to a chloroplast photosystem II. Relationships: is a type of protein-containing complex binding [GO:0044877] References: PMID:17400553